{
  "gene_name": "Small ribosomal subunit protein uS11m",
  "term_id": "GO:0003735",
  "gene": "UniProtKB:P82912",
  "term_label": "structural constituent of ribosome",
  "gene_symbol": "MRPS11"
}